positive regulation of glycogen catabolic process [GO:0045819] (biological process) Relationships: is a type of GO:0005981; is a type of positive regulation of catabolic process [GO:0009896]; is a type of positive regulation of glycogen metabolic process [GO:0070875]; positively regulates glycogen catabolic process [GO:0005980] Sources: GOC:go_curators Also known as: positive regulation of glycogen breakdown, positive regulation of glycogen catabolism, positive regulation of glycogen degradation, positive regulation of glycogenolysis, up regulation of glycogen catabolic process, up-regulation of glycogen catabolic process, upregulation of glycogen catabolic process, activation of glycogen catabolic process, stimulation of glycogen catabolic process Definition: Any process that activates or increases the frequency, rate or extent of the chemical reactions and pathways resulting in the breakdown of glycogen.